{
  "gene_symbol": "SEC16A",
  "gene": "UniProtKB:O15027",
  "gene_name": "Protein transport protein Sec16A",
  "term_id": "GO:0006888",
  "term_label": "endoplasmic reticulum to Golgi vesicle-mediated transport"
}